{
  "gene_name": "Sphingomyelin synthase-related protein 1",
  "gene_symbol": "SAMD8",
  "term_label": "plasma membrane",
  "gene": "UniProtKB:Q96LT4",
  "term_id": "GO:0005886"
}